gallate catabolic process via gallate dioxygenase activity [GO:0019398] (biological process) Definition: The chemical reactions and pathways resulting in the breakdown of gallate, the anion of gallic acid, where the first step is the conversion of gallate to (1E)-4-oxobut-1-ene-1,2,4-tricarboxylate catalyzed by gallate dioxygenase. Sources: GOC:bf, GOC:jl Also known as: gallate catabolic process via 4-carboxy-2-hydroxhexa-2,3-dienedioate, gallate breakdown via 4-carboxy-2-hydroxhexa-2,3-dienedioate, gallate degradation via 4-carboxy-2-hydroxhexa-2,3-dienedioate, gallic acid catabolic process via 4-carboxy-2-hydroxhexa-2,3-dienedioate, gallic acid catabolism via 4-carboxy-2-hydroxhexa-2,3-dienedioate Relationships: is a type of aerobic gallate catabolic process [GO:0042195]; BFO_0000051 gallate dioxygenase activity [GO:0036238]